{
  "term_label": "regulation of cilium movement",
  "gene_symbol": "CCDC65",
  "gene_name": "Dynein regulatory complex subunit 2",
  "gene": "UniProtKB:Q8IXS2",
  "term_id": "GO:0003352"
}